TAM protein secretion complex [GO:0097347] (CC) References: PMID:22466966 Sources: GOC:am Definition: A heterooligomeric protein complex that spans the bacterial periplasm and enables the secretion of adhesin proteins in Gram-negative bacteria. In Citrobacter rodentium, Salmonella enterica and Escherichia coli, the TAM complex consists of an Omp85-family protein, TamA, in the outer membrane and TamB in the inner membrane. Relationships: is a type of protein-containing complex [GO:0032991] Also known as: translocation and assembly module protein complex